{
  "gene_symbol": "OSR1",
  "gene_name": "Protein odd-skipped-related 1",
  "term_label": "RNA polymerase II transcription regulatory region sequence-specific DNA binding",
  "term_id": "GO:0000977",
  "gene": "UniProtKB:Q8TAX0"
}